negative regulation of translational initiation in response to stress [GO:0032057] (biological process) Sources: GOC:mah Subtypes: negative regulation of translational initiation in response to osmotic stress [GO:0032063], negative regulation of translation in response to oxidative stress [GO:0032938], GO:0036495, negative regulation of translational initiation in response to starvation [GO:0071263], negative regulation of cytoplasmic translational initiation in response to stress [GO:1990625] Also known as: down regulation of translation initiation in response to stress, down-regulation of translation initiation in response to stress, downregulation of translation initiation in response to stress, inhibition of translation initiation in response to stress Definition: Any process that stops, prevents or reduces the rate of translation initiation as a result of a stimulus indicating the organism is under stress. Relationships: is a type of negative regulation of translational initiation [GO:0045947]; is part of GO:0006950